{
  "term_id": "GO:1990180",
  "gene": "UniProtKB:Q96Q11",
  "gene_symbol": "TRNT1",
  "term_label": "mitochondrial tRNA 3'-end processing",
  "gene_name": "CCA tRNA nucleotidyltransferase 1, mitochondrial"
}